{
  "gene_name": "Endothelial zinc finger protein induced by tumor necrosis factor alpha",
  "term_id": "GO:0006357",
  "gene_symbol": "ZNF71",
  "gene": "UniProtKB:Q9NQZ8",
  "term_label": "regulation of transcription by RNA polymerase II"
}